regulation of tongue muscle cell differentiation [GO:2001035] (biological process) Definition: Any process that modulates the frequency, rate or extent of tongue muscle cell differentiation. Subtypes: negative regulation of tongue muscle cell differentiation [GO:2001036], positive regulation of tongue muscle cell differentiation [GO:2001037] Sources: GOC:obol Relationships: is_a GO:1902809; regulates GO:0035981